{
  "term_id": "GO:0005739",
  "gene_name": "Sterol 26-hydroxylase, mitochondrial",
  "term_label": "mitochondrion",
  "gene": "UniProtKB:Q02318",
  "gene_symbol": "CYP27A1"
}